D-glycero-beta-D-manno-heptose 1,7-bisphosphate 7-phosphatase activity [GO:0034200] (molecular function) Relationships: is a type of phosphatase activity [GO:0016791] Also known as: D,D-heptose 1,7-bisphosphate phosphatase activity References: PMID:11279237 Sources: RHEA:28518 Definition: Catalysis of the reaction: D-glycero-beta-D-manno-heptose 1,7-bisphosphate + H2O = D-glycero-beta-D-manno-heptose 1-phosphate + phosphate.